{
  "term_label": "mitochondrial electron transport, NADH to ubiquinone",
  "gene_name": "NADH dehydrogenase [ubiquinone] flavoprotein 2, mitochondrial",
  "term_id": "GO:0006120",
  "gene_symbol": "NDUFV2",
  "gene": "UniProtKB:P19404"
}